L-histidine:2-oxoglutarate aminotransferase activity [GO:0008110] (MF) Relationships: is a type of transaminase activity [GO:0008483] Sources: EC:2.6.1.38, RHEA:16565 Definition: Catalysis of the reaction: 2-oxoglutarate + L-histidine = 3-(imidazol-5-yl)pyruvate + L-glutamate. Also known as: histidine aminotransferase activity, histidine transaminase activity, histidine-2-oxoglutarate aminotransferase activity